{
  "term_id": "UNKNOWN:0003",
  "gene_symbol": "GPR158",
  "term_label": "Unknown cellular component",
  "gene_name": "Probable G-protein coupled receptor 158",
  "gene": "UniProtKB:Q5T848"
}